lycopene biosynthetic process [GO:1901177] (biological process) Relationships: is_a carotene biosynthetic process [GO:0016120] Sources: GOC:TermGenie, GOC:yaf, UniPathway:UPA00803 Also known as: lycopene anabolism, lycopene biosynthesis, lycopene formation, lycopene synthesis Definition: The chemical reactions and pathways resulting in the formation of lycopene.